{
  "term_id": "UNKNOWN:0001",
  "gene_name": "Rab11 family-interacting protein 3",
  "gene_symbol": "RAB11FIP3",
  "gene": "UniProtKB:O75154",
  "term_label": "Unknown molecular function"
}